acryloyl-CoA reductase (NADPH) activity [GO:0043957] (molecular function) Definition: Catalysis of the reaction: acryloyl-CoA + NADPH + H+ = propionyl-CoA + NADP+. Note: Note that this function is one of the activities of the trifunctional enzyme propionyl-coenzyme A synthase. See PMID:11821399. References: PMID:11821399 Sources: GOC:jl, RHEA:26454 Also known as: AMP-dependent synthetase and ligase, AMP-dependent synthetase and ligase:enoyl-CoA hydratase/isomerase, acetyl-coenzyme A synthetase, acetyl-coenzyme A synthetase/GroES-like domain, enoyl-CoA hydratase/isomerase, acrylyl-CoA reductase (NADPH) activity Relationships: is a type of oxidoreductase activity, acting on the CH-CH group of donors, NAD or NADP as acceptor [GO:0016628]